{
  "term_label": "telomerase RNA binding",
  "gene_name": "Telomerase protein component 1",
  "gene": "UniProtKB:Q99973",
  "term_id": "GO:0070034",
  "gene_symbol": "TEP1"
}